{
  "gene_symbol": "PRDM1",
  "gene_name": "PR domain zinc finger protein 1",
  "term_id": "GO:0006357",
  "gene": "UniProtKB:O75626",
  "term_label": "regulation of transcription by RNA polymerase II"
}